cardiac muscle adaptation [GO:0014887] (biological process) Definition: The process in which cardiac muscle adapts, with consequent modifications to structural and/or functional phenotypes, in response to a stimulus. Stimuli include contractile activity, loading conditions, substrate supply, and environmental factors. Sources: GOC:mtg_muscle Also known as: cardiac muscle plasticity Relationships: is a type of striated muscle adaptation [GO:0014888] Subtypes: GO:0014898, cardiac muscle atrophy [GO:0014899] Regulation: regulated by GO:0010612; positively regulated by positive regulation of cardiac muscle adaptation [GO:0010615]; negatively regulated by negative regulation of cardiac muscle adaptation [GO:0010616]